positive regulation of foraging behavior [GO:1903370] (biological process) Definition: Any process that activates or increases the frequency, rate or extent of foraging behavior. Also known as: up regulation of foraging behavior, up-regulation of foraging behavior, upregulation of foraging behavior, activation of foraging behavior References: PMID:8677262 Sources: GOC:TermGenie, GOC:mr, GO_REF:0000058 Relationships: is a type of positive regulation of behavior [GO:0048520]; is a type of regulation of foraging behavior [GO:1903368]; positively regulates foraging behavior [GO:0060756]